ribose-5-phosphate adenylyltransferase activity [GO:0047345] (molecular function) Sources: EC:2.7.7.35, RHEA:14529 Relationships: is a type of adenylyltransferase activity [GO:0070566] Also known as: ADP:ribose-5-phosphate adenylyltransferase activity, ADP ribose phosphorylase activity, ADP-ribose phosphorylase activity, ADP:D-ribose-5-phosphate adenylyltransferase activity, adenosine diphosphoribose phosphorylase activity Definition: Catalysis of the reaction: D-ribose 5-phosphate + ADP + H+ = ADP-ribose + phosphate.